catalase activity [GO:0004096] (MF) Sources: EC:1.11.1.6 Relationships: is a type of peroxidase activity [GO:0004601] Also known as: catalase reaction, bacterial catalase-peroxidase activity, haem catalase activity, heme catalase activity, manganese catalase activity, CAT, caperase activity, catalase-peroxidase activity, equilase activity, hydrogen-peroxide:hydrogen-peroxide oxidoreductase activity, optidase activity Definition: Catalysis of the reaction: 2 hydrogen peroxide = O2 + 2 H2O. Regulation: positively regulated by GO:1902553